caudate nucleus development [GO:0021757] (biological process) Relationships: is a type of GO:0048857; is part of striatum development [GO:0021756] Definition: The progression of the caudate nucleus over time from its initial formation until its mature state. The caudate nucleus is the C-shaped structures of the striatum containing input neurons involved with control of voluntary movement in the brain. Sources: GOC:cls, GOC:dgh, GOC:dph, GOC:jid, GO_REF:0000021